{
  "term_id": "GO:0008375",
  "gene_symbol": "GCNT4",
  "term_label": "acetylglucosaminyltransferase activity",
  "gene": "UniProtKB:Q9P109",
  "gene_name": "Beta-1,3-galactosyl-O-glycosyl-glycoprotein beta-1,6-N-acetylglucosaminyltransferase 4"
}